{
  "term_label": "Unknown molecular function",
  "term_id": "UNKNOWN:0001",
  "gene": "UniProtKB:Q4AC94",
  "gene_name": "C2 domain-containing protein 3",
  "gene_symbol": "C2CD3"
}